{
  "term_id": "GO:0005634",
  "gene_name": "Homeobox protein Hox-A6",
  "gene": "UniProtKB:P31267",
  "term_label": "nucleus",
  "gene_symbol": "HOXA6"
}